{
  "gene_name": "Connector enhancer of kinase suppressor of ras 1",
  "term_id": "GO:0007167",
  "term_label": "enzyme-linked receptor protein signaling pathway",
  "gene": "UniProtKB:Q969H4",
  "gene_symbol": "CNKSR1"
}